{
  "term_label": "perinuclear endoplasmic reticulum",
  "gene_symbol": "OSBPL2",
  "gene": "UniProtKB:Q9H1P3",
  "gene_name": "Oxysterol-binding protein-related protein 2",
  "term_id": "GO:0097038"
}